{
  "gene_symbol": "B3GALNT2",
  "gene_name": "UDP-GalNAc:beta-1,3-N-acetylgalactosaminyltransferase 2",
  "term_label": "protein O-linked glycosylation",
  "gene": "UniProtKB:Q8NCR0",
  "term_id": "GO:0006493"
}